specification of animal organ axis polarity [GO:0010084] (biological process) Sources: GOC:tb Relationships: is a type of specification of axis polarity [GO:0065001]; is part of animal organ morphogenesis [GO:0009887] Definition: The process in which the polarity of an animal organ axis is specified.